{
  "gene_name": "Sodium-dependent proline transporter",
  "gene_symbol": "SLC6A7",
  "gene": "UniProtKB:Q99884",
  "term_id": "GO:0015824",
  "term_label": "proline transport"
}